{
  "gene_symbol": "RNFT1",
  "term_label": "endoplasmic reticulum",
  "gene_name": "E3 ubiquitin-protein ligase RNFT1",
  "gene": "UniProtKB:Q5M7Z0",
  "term_id": "GO:0005783"
}